regulation of T-helper cell differentiation [GO:0045622] (biological process) Definition: Any process that modulates the frequency, rate or extent of T-helper cell differentiation. Subtypes: GO:0045623, positive regulation of T-helper cell differentiation [GO:0045624], regulation of T-helper 1 cell differentiation [GO:0045625], regulation of T-helper 2 cell differentiation [GO:0045628], regulation of T-helper 17 cell differentiation [GO:2000319] Sources: GOC:go_curators Also known as: regulation of T-helper cell development Note: Note that immunologists typically use the word 'development' to refer to cells of B or T cell lineages undergoing the process that GO describes as 'cell differentiation'. Relationships: is a type of regulation of immune effector process [GO:0002697]; is a type of regulation of CD4-positive, alpha-beta T cell differentiation [GO:0043370]; is a type of regulation of immune response [GO:0050776]; RO_0002211 T-helper cell differentiation [GO:0042093]